{
  "gene_name": "Recombining binding protein suppressor of hairless",
  "gene": "UniProtKB:Q06330",
  "term_id": "GO:0000978",
  "gene_symbol": "RBPJ",
  "term_label": "RNA polymerase II cis-regulatory region sequence-specific DNA binding"
}